{
  "term_id": "UNKNOWN:0003",
  "gene": "UniProtKB:Q86TD4",
  "gene_symbol": "SRL",
  "term_label": "Unknown cellular component",
  "gene_name": "Sarcalumenin"
}